{
  "gene": "UniProtKB:P0CG37",
  "term_label": "nodal binding",
  "gene_symbol": "CFC1",
  "gene_name": "Cryptic protein",
  "term_id": "GO:0038100"
}